{
  "gene_symbol": "TMEM231",
  "gene_name": "Transmembrane protein 231",
  "gene": "UniProtKB:Q9H6L2",
  "term_id": "GO:0060271",
  "term_label": "cilium assembly"
}